{
  "gene": "UniProtKB:Q96DN5",
  "gene_symbol": "TBC1D31",
  "gene_name": "TBC1 domain family member 31",
  "term_id": "GO:0060271",
  "term_label": "cilium assembly"
}